{
  "gene_symbol": "RAB12",
  "gene_name": "Ras-related protein Rab-12",
  "term_id": "GO:0003924",
  "term_label": "GTPase activity",
  "gene": "UniProtKB:Q6IQ22"
}